{
  "gene": "UniProtKB:P53667",
  "gene_name": "LIM domain kinase 1",
  "gene_symbol": "LIMK1",
  "term_label": "cytoplasm",
  "term_id": "GO:0005737"
}